{
  "gene_name": "Netrin receptor DCC",
  "gene": "UniProtKB:P43146",
  "term_label": "cell-cell adhesion",
  "gene_symbol": "DCC",
  "term_id": "GO:0098609"
}